{
  "gene_name": "Inositol-trisphosphate 3-kinase A",
  "term_label": "inositol phosphate biosynthetic process",
  "gene_symbol": "ITPKA",
  "term_id": "GO:0032958",
  "gene": "UniProtKB:P23677"
}